{
  "term_label": "sarcomere",
  "gene_name": "Leucine-rich repeat-containing protein 10",
  "gene": "UniProtKB:Q5BKY1",
  "term_id": "GO:0030017",
  "gene_symbol": "LRRC10"
}